RNA polymerase II CTD heptapeptide repeat S5 phosphatase activity [GO:0180007] (molecular function) References: PMID:22622228 Relationships: is a type of GO:0008420 Also known as: RNA polymerase II C-terminal domain S5 phosphatase activity Definition: Catalysis of the reaction: RNA polymerase II large subunit CTD heptapeptide repeat--phospho-L-serine (consensus YSPTSPS)(position 5) + H2O = RNA polymerase II large subunit + phosphate.